3-methylbut-2-enoyl-CoA(4-) catabolic process [GO:1902199] (biological process) References: PMID:11231285 Sources: GOC:TermGenie Also known as: 3-methylbut-2-enoyl-CoA(4-) breakdown, 3-methylbut-2-enoyl-CoA(4-) catabolism, 3-methylbut-2-enoyl-CoA(4-) degradation Definition: The chemical reactions and pathways resulting in the breakdown of 3-methylbut-2-enoyl-CoA(4-). Relationships: is a type of GO:0036115; is_a 3-methylbut-2-enoyl-CoA(4-) metabolic process [GO:1902198]